{
  "gene": "UniProtKB:Q9NRP2",
  "gene_name": "COX assembly mitochondrial protein 2 homolog",
  "gene_symbol": "CMC2",
  "term_id": "UNKNOWN:0002",
  "term_label": "Unknown biological process"
}